regulation of cellular hyperosmotic salinity response [GO:1900069] (biological process) Definition: Any process that modulates the frequency, rate or extent of cellular hyperosmotic salinity response. References: PMID:16278455 Sources: GOC:TermGenie, GOC:dgf Also known as: regulation of cellular response to hyperosmotic salt stress Relationships: is_a GO:0106049; is_a GO:1901000; regulates cellular hyperosmotic salinity response [GO:0071475] Subtypes: GO:1900070